FMN reductase complex [GO:1990202] (cellular component) Definition: A protein complex capable of FMN reductase activity. Reduces FMN to FMNH2 in a NAD(P)H-dependent manner. In E.coli, consists of a SsuE dimer. References: PMID:10480865, PMID:16997955 Sources: GOC:bhm Also known as: flavin oxidoreductase complex, NAD(P)H-dependent, FMN reductase complex, NAD(P)H-dependent, SsuE complex, FMN oxidoreductase complex, NAD(P)H-dependent Relationships: is_a oxidoreductase complex [GO:1990204]; is part of cytosol [GO:0005829]